global genome nucleotide-excision repair [GO:0070911] (biological process) Relationships: is a type of nucleotide-excision repair [GO:0006289] References: PMID:10197977, PMID:18794354 Also known as: GG-NER, GGR, global genome NER, global genomic nucleotide-excision repair, global genomic repair Definition: The nucleotide-excision repair process in which DNA lesions are removed from nontranscribed strands and from transcriptionally silent regions over the entire genome.